asparaginase activity [GO:0004067] (molecular function) Also known as: L-asparaginase activity, L-asparagine amidohydrolase activity, alpha-asparaginase activity, asparaginase II, colaspase activity, crasnitin, elspar, leunase activity Relationships: is a type of amidase activity [GO:0004040] Sources: EC:3.5.1.1 Definition: Catalysis of the reaction: L-asparagine + H2O = L-aspartate + NH4+.